{
  "gene_symbol": "H1-6",
  "gene_name": "Histone H1t",
  "gene": "UniProtKB:P22492",
  "term_id": "GO:0007283",
  "term_label": "spermatogenesis"
}